lymph vessel morphogenesis [GO:0036303] (biological process) Relationships: is a type of anatomical structure morphogenesis [GO:0009653]; is part of lymph vessel development [GO:0001945] References: PMID:18093989 Sources: GOC:BHF, GOC:gr Definition: The process in which the anatomical structures of lymph vessels are generated and organized. The lymph vessel is the vasculature carrying lymph.